{
  "term_id": "UNKNOWN:0001",
  "term_label": "Unknown molecular function",
  "gene_name": "ER membrane protein complex subunit 4",
  "gene_symbol": "EMC4",
  "gene": "UniProtKB:Q5J8M3"
}